{
  "term_id": "UNKNOWN:0003",
  "term_label": "Unknown cellular component",
  "gene_name": "Arylsulfatase J",
  "gene_symbol": "ARSJ",
  "gene": "UniProtKB:Q5FYB0"
}